pole cell formation [GO:0007279] (biological process) Note: See also the Cell Ontology term 'pole cell ; CL:0000301'. Relationships: is a type of GO:0003006; is a type of cellularization [GO:0007349]; is part of pole cell development [GO:0007277] Definition: Formation of a small group of cells (pole cells) at the posterior pole of the insect blastula. They are the first cells to cellularize after the arrival of nuclei at the end of the syncytial blastula stage and are the precursors to the insect germ cells. References: PMID:9988212 Sources: GOC:bf